{
  "gene": "UniProtKB:O95749",
  "term_id": "UNKNOWN:0003",
  "gene_name": "Geranylgeranyl pyrophosphate synthase",
  "gene_symbol": "GGPS1",
  "term_label": "Unknown cellular component"
}